permeabilization of host organelle membrane involved in viral entry into host cell [GO:0039665] (biological process) Definition: Induction of organellar membrane permeabilization triggered by an interaction between the host membrane and a membrane-penetration protein associated with a viral capsid. Results in release of the virus contents from an organelle into the host cell cytoplasm. Sources: GOC:bf, GOC:jl, UniProtKB-KW:KW-1173, VZ:985 Also known as: viral penetration via host endosomal membrane disruption by virus, viral penetration via perforation of host organellar membrane by virus, viral penetration via permeabilization of host organellar membrane, viral entry into host cell via permeabilization of host organelle membrane, viral membrane-penetration protein Relationships: is a type of viral process [GO:0016032]; is part of symbiont entry into host cell via permeabilization of host membrane [GO:0140267] Subtypes: GO:0075502, GO:0075504